{
  "term_label": "poly(A) RNA polymerase activity",
  "gene": "UniProtKB:Q5XG87",
  "gene_name": "Terminal nucleotidyltransferase 4A",
  "gene_symbol": "TENT4A",
  "term_id": "GO:1990817"
}